{
  "term_id": "UNKNOWN:0001",
  "gene": "UniProtKB:Q6ZU35",
  "gene_name": "Capping protein-inhibiting regulator of actin dynamics",
  "gene_symbol": "CRACD",
  "term_label": "Unknown molecular function"
}